{
  "term_label": "mitochondrial inner membrane",
  "gene_symbol": "ETFDH",
  "gene": "UniProtKB:Q16134",
  "gene_name": "Electron transfer flavoprotein-ubiquinone oxidoreductase, mitochondrial",
  "term_id": "GO:0005743"
}